{
  "gene": "UniProtKB:Q7Z5H5",
  "gene_symbol": "VN1R4",
  "term_id": "UNKNOWN:0002",
  "term_label": "Unknown biological process",
  "gene_name": "Vomeronasal type-1 receptor 4"
}